integrated stress response signaling [GO:0140467] (BP) Also known as: ISR Definition: The series of molecular signals generated in response to diverse stress stimuli required to restore cellular homeostasis. The core event in this pathway is the phosphorylation of eIF2 alpha by one of four members of the eIF2a kinase family (EIF2AK1/HRI, EIF2AK2/PKR, EIF2AK3/PERK and EIF2AK4/GCN2), which leads to a decrease in global protein synthesis and the induction of selected genes, including the transcription factor ATF4, that together promote cellular recovery. Subtypes: GO:0036499, PKR/eIFalpha signaling [GO:0039585], HRI-mediated signaling [GO:0140468], GO:0140469 Relationships: is a type of GO:0033554; is a type of intracellular signaling cassette [GO:0141124] References: PMID:27629041